{
  "gene": "UniProtKB:Q9H4X1",
  "term_label": "protein kinase binding",
  "gene_name": "Regulator of cell cycle RGCC",
  "term_id": "GO:0019901",
  "gene_symbol": "RGCC"
}